{
  "gene_symbol": "STAT5B",
  "gene_name": "Signal transducer and activator of transcription 5B",
  "gene": "UniProtKB:P51692",
  "term_id": "GO:0090575",
  "term_label": "RNA polymerase II transcription regulator complex"
}